{
  "gene": "UniProtKB:Q96EY5",
  "term_label": "regulation of epidermal growth factor receptor signaling pathway",
  "gene_name": "Multivesicular body subunit 12A",
  "gene_symbol": "MVB12A",
  "term_id": "GO:0042058"
}